regulation of mitotic actomyosin contractile ring contraction [GO:1903471] (biological process) Relationships: is a type of regulation of actomyosin contractile ring contraction [GO:0031991]; is a type of regulation of mitotic cytokinetic process [GO:1903436]; regulates mitotic actomyosin contractile ring contraction [GO:1902404] References: PMID:1234 Sources: GOC:TermGenie, GOC:mtg_cell_cycle, GO_REF:0000058 Subtypes: GO:1903472, GO:1903473 Definition: Any process that modulates the frequency, rate or extent of mitotic actomyosin contractile ring contraction. Also known as: regulation of contractile ring contraction involved in cell cycle cytokinesis involved in mitotic cell cycle, regulation of cytokinesis, actomyosin ring contraction involved in mitotic cell cycle, regulation of mitotic actomyosin contractile ring constriction